{
  "gene_symbol": "VASP",
  "gene": "UniProtKB:P50552",
  "term_label": "actin polymerization or depolymerization",
  "term_id": "GO:0008154",
  "gene_name": "Vasodilator-stimulated phosphoprotein"
}